{
  "term_id": "GO:0030593",
  "gene_symbol": "CXCL6",
  "term_label": "neutrophil chemotaxis",
  "gene": "UniProtKB:P80162",
  "gene_name": "C-X-C motif chemokine 6"
}